response to jasmonic acid stimulus involved in jasmonic acid and ethylene-dependent systemic resistance [GO:0032260] (biological process) Definition: Any process that results in a change in state or activity of a cell or an organism (in terms of movement, secretion, enzyme production, gene expression, etc.) as a result of a jasmonic acid stimulus received in the context of the jasmonic acid- and ethylene (ethene)-dependent process that confers broad spectrum systemic resistance to disease in response to wounding or a pathogen. Sources: GOC:mah Also known as: response to jasmonic acid stimulus during jasmonic acid and ethylene-dependent systemic resistance Relationships: is a type of response to jasmonic acid [GO:0009753]; is part of jasmonic acid and ethylene-dependent systemic resistance [GO:0009861]